regulation of endoplasmic reticulum unfolded protein response [GO:1900101] (biological process) Definition: Any process that modulates the frequency, rate or extent of endoplasmic reticulum unfolded protein response. Subtypes: negative regulation of endoplasmic reticulum unfolded protein response [GO:1900102], positive regulation of endoplasmic reticulum unfolded protein response [GO:1900103], GO:1903891, regulation of IRE1-mediated unfolded protein response [GO:1903894], regulation of PERK-mediated unfolded protein response [GO:1903897] Also known as: regulation of ER unfolded protein response, regulation of erUPR, regulation of SREBP-mediated signalling pathway Relationships: is a type of regulation of intracellular signal transduction [GO:1902531]; is a type of regulation of response to endoplasmic reticulum stress [GO:1905897]; regulates endoplasmic reticulum unfolded protein response [GO:0030968] Sources: GOC:TermGenie